secondary active cyanate transmembrane transporter activity [GO:0015541] (molecular function) Definition: Enables the transfer of cyanate from one side of a membrane to the other. Also known as: cyanate porter activity Sources: TC:2.A.1.17.1 Relationships: is_a cyanate transmembrane transporter activity [GO:0015110]; is_a secondary active transmembrane transporter activity [GO:0015291]